ribonuclease U2 activity [GO:0033899] (molecular function) Relationships: is a type of RNA endonuclease activity [GO:0004521]; is a type of GO:0016849 Sources: EC:4.6.1.20 Also known as: pleospora RNase activity, purine specific endoribonuclease activity, purine-specific RNase activity, purine-specific ribonuclease activity, ribonuclease (purine) activity, trichoderma koningi RNase III activity, RNase U2 activity Definition: Catalysis of the two-stage endonucleolytic cleavage to nucleoside 3'-phosphates and 3'-phosphooligonucleotides ending in Ap or Gp with 2',3'-cyclic phosphate intermediates.